ERBB2 signaling pathway [GO:0038128] (biological process) References: PMID:16460914 Sources: GOC:jc Subtypes: ERBB2-ERBB3 signaling pathway [GO:0038133], ERBB2-EGFR signaling pathway [GO:0038134], GO:0038135 Relationships: is a type of ERBB signaling pathway [GO:0038127] Definition: The series of molecular signals initiated by binding of a ligand to the tyrosine kinase receptor ERBB2 on the surface of a cell. The pathway ends with regulation of a downstream cellular process, e.g. transcription. ERBB2 receptors are themselves unable to bind to ligands, but act as a signal-amplifying tyrosine kinase within a heterodimeric pair. Also known as: ERBB2 signalling pathway, HER2 signaling pathway, NEU signaling, receptor tyrosine-protein kinase erbB-2 signaling pathway